{
  "gene_name": "Cyclin-I",
  "term_label": "cyclin-dependent protein serine/threonine kinase regulator activity",
  "term_id": "GO:0016538",
  "gene": "UniProtKB:Q14094",
  "gene_symbol": "CCNI"
}